voltage-gated calcium channel activity involved in regulation of cytosolic calcium levels [GO:0099511] (molecular function) Subtypes: GO:0099626, voltage-gated calcium channel activity involved in regulation of postsynaptic cytosolic calcium levels [GO:1905057] Sources: GOC:dos Definition: Regulation of cytosolic calcium ion concentrations via the directed movement of calcium ions across the plasma-membrane into the cytosol via the action of a voltage-gated calcium ion channel. Relationships: is a type of voltage-gated calcium channel activity [GO:0005245]; is part of regulation of cytosolic calcium ion concentration [GO:0051480]